{
  "term_id": "GO:0005789",
  "gene_name": "Selenoprotein K",
  "term_label": "endoplasmic reticulum membrane",
  "gene": "UniProtKB:Q9Y6D0",
  "gene_symbol": "SELENOK"
}